{
  "term_id": "GO:0016192",
  "term_label": "vesicle-mediated transport",
  "gene_name": "Kinesin-like protein KIF1C",
  "gene": "UniProtKB:O43896",
  "gene_symbol": "KIF1C"
}